{
  "term_label": "sphingolipid biosynthetic process",
  "term_id": "GO:0030148",
  "gene": "UniProtKB:B0YJ81",
  "gene_name": "Very-long-chain (3R)-3-hydroxyacyl-CoA dehydratase 1",
  "gene_symbol": "HACD1"
}